{
  "term_label": "nucleus",
  "gene_symbol": "AHNAK2",
  "gene": "UniProtKB:Q8IVF2",
  "term_id": "GO:0005634",
  "gene_name": "Protein AHNAK2"
}